{
  "term_id": "GO:0042605",
  "gene_name": "HLA class I histocompatibility antigen, alpha chain E",
  "term_label": "peptide antigen binding",
  "gene_symbol": "HLA-E",
  "gene": "UniProtKB:P13747"
}